protein folding chaperone complex [GO:0101031] (cellular component) Also known as: chaperone complex References: PMID:21855797 Sources: GOC:bhm Note: An example of this is HSP90AB1 in human (P08238) in PMID:21855797 (inferred from direct assay). Definition: A protein complex required for the non-covalent folding or unfolding, maturation, stabilization or assembly or disassembly of macromolecular structures. Usually active during or immediately after completion of translation. Many chaperone complexes contain heat shock proteins. Subtypes: chaperonin-containing T-complex [GO:0005832], chaperonin ATPase complex [GO:0016465], Ig heavy chain-bound endoplasmic reticulum chaperone complex [GO:0034664], mitochondrial respiratory chain complex IV pre-assembly complex [GO:0062011], large ribosomal subunit pre-assembly complex [GO:0140714], GO:1990565 Relationships: is_a intracellular protein-containing complex [GO:0140535]